5-diphosphoinositol pentakisphosphate 1-kinase activity [GO:0033857] (molecular function) Relationships: is a type of diphosphoinositol pentakisphosphate kinase activity [GO:0000829] Sources: EC:2.7.4.24 Definition: Catalysis of the reaction: ATP + 1D-myo-inositol 5-diphosphate pentakisphosphate = ADP + 1D-myo-inositol bisdiphosphate tetrakisphosphate. Also known as: diphosphoinositol-pentakisphosphate kinase activity, inositol heptakisphosphate 1-kinase activity, PP-IP5 kinase activity, PP-InsP5 kinase activity, PPIP5K